{
  "gene_symbol": "CFC1B",
  "gene_name": "Cryptic family protein 1B",
  "term_label": "heart development",
  "gene": "UniProtKB:P0CG36",
  "term_id": "GO:0007507"
}